{
  "term_id": "UNKNOWN:0003",
  "gene_symbol": "MTARC1",
  "gene_name": "Mitochondrial amidoxime-reducing component 1",
  "term_label": "Unknown cellular component",
  "gene": "UniProtKB:Q5VT66"
}